{
  "term_id": "UNKNOWN:0001",
  "gene_name": "Ubiquinol-cytochrome-c reductase complex assembly factor 6",
  "term_label": "Unknown molecular function",
  "gene_symbol": "UQCC6",
  "gene": "UniProtKB:Q69YU5"
}